myosin II filament organization [GO:0031038] (biological process) Relationships: is a type of myosin filament organization [GO:0031033] Regulation: regulated by regulation of myosin II filament organization [GO:0043519]; negatively regulated by negative regulation of myosin II filament organization [GO:1904900]; positively regulated by positive regulation of myosin II filament organization [GO:1904901] Definition: A process that is carried out at the cellular level which results in the assembly, arrangement of constituent parts, or disassembly of a bipolar filament composed of myosin II molecules. Subtypes: myosin II filament assembly [GO:0031036], GO:0031037 Also known as: myosin II filament organisation, myosin II filament assembly or disassembly, myosin II polymerization or depolymerization Sources: GOC:mah